positive regulation of mismatch repair [GO:0032425] (biological process) Definition: Any process that activates or increases the frequency, rate or extent of mismatch repair. Sources: GOC:vk Also known as: up regulation of mismatch repair, up-regulation of mismatch repair, upregulation of mismatch repair, activation of mismatch repair, stimulation of mismatch repair Relationships: is a type of regulation of mismatch repair [GO:0032423]; is_a positive regulation of DNA repair [GO:0045739]; positively regulates mismatch repair [GO:0006298]